{
  "term_id": "GO:0048741",
  "gene_symbol": "MYORG",
  "gene_name": "Myogenesis-regulating glycosidase",
  "term_label": "skeletal muscle fiber development",
  "gene": "UniProtKB:Q6NSJ0"
}